{
  "gene_name": "Chromodomain-helicase-DNA-binding protein 2",
  "term_id": "GO:0016887",
  "term_label": "ATP hydrolysis activity",
  "gene": "UniProtKB:O14647",
  "gene_symbol": "CHD2"
}